positive regulation of mitotic actomyosin contractile ring assembly [GO:1903501] (BP) References: PMID:18256290 Sources: GOC:TermGenie, GOC:al, GOC:mtg_cell_cycle, GOC:vw, GO_REF:0000058 Also known as: positive regulation of actomyosin contractile ring assembly involved in cytokinesis after mitosis, positive regulation of contractile ring assembly involved in mitotic cytokinesis, positive regulation of cytokinesis, actomyosin contractile ring assembly involved in mitotic cytokinesis, positive regulation of mitotic cytokinesis, actomyosin contractile ring assembly, up regulation of actomyosin contractile ring assembly involved in cytokinesis after mitosis, up regulation of contractile ring assembly involved in mitotic cytokinesis, up regulation of cytokinesis, actomyosin contractile ring assembly involved in mitotic cytokinesis, up regulation of mitotic actomyosin contractile ring assembly, up-regulation of actomyosin contractile ring assembly involved in cytokinesis after mitosis, up-regulation of contractile ring assembly involved in mitotic cytokinesis, up-regulation of cytokinesis, actomyosin contractile ring assembly involved in mitotic cytokinesis, up-regulation of mitotic actomyosin contractile ring assembly, upregulation of actomyosin contractile ring assembly involved in cytokinesis after mitosis, upregulation of contractile ring assembly involved in mitotic cytokinesis, upregulation of cytokinesis, actomyosin contractile ring assembly involved in mitotic cytokinesis, upregulation of mitotic actomyosin contractile ring assembly, activation of actomyosin contractile ring assembly involved in cytokinesis after mitosis, activation of contractile ring assembly involved in mitotic cytokinesis, activation of cytokinesis, actomyosin contractile ring assembly involved in mitotic cytokinesis, activation of mitotic actomyosin contractile ring assembly Relationships: is a type of GO:1903438; is a type of regulation of mitotic actomyosin contractile ring assembly [GO:1903499]; is a type of positive regulation of cytokinesis, actomyosin contractile ring assembly [GO:2000433]; positively regulates mitotic actomyosin contractile ring assembly [GO:1903475] Definition: Any process that activates or increases the frequency, rate or extent of mitotic actomyosin contractile ring assembly.